{
  "term_label": "nucleus",
  "gene": "UniProtKB:Q8WUB8",
  "gene_name": "PHD finger protein 10",
  "gene_symbol": "PHF10",
  "term_id": "GO:0005634"
}